alpha9-beta1 integrin-ADAM12 complex [GO:0071068] (cellular component) Relationships: is a type of plasma membrane protein complex [GO:0098797] References: PMID:10944520 Also known as: ITGA9-ITGB1-ADAM12 complex Definition: A protein complex that consists of an alpha9-beta1 integrin complex bound to the transmembrane metallopeptidase ADAM12.